positive regulation of viral entry into host cell [GO:0046598] (biological process) Also known as: positive regulation of viral penetration into host cell Subtypes: GO:1903915 Relationships: is a type of regulation of viral entry into host cell [GO:0046596]; is_a positive regulation by symbiont of entry into host [GO:0075294]; is a type of GO:1903902; positively regulates symbiont entry into host cell [GO:0046718] Definition: Any process that activates or increases the frequency, rate or extent of the introduction of viral entry into the host cell. Sources: GOC:jl